{
  "gene": "UniProtKB:Q15831",
  "term_label": "nucleus",
  "gene_name": "Serine_threonine-protein kinase STK11",
  "term_id": "GO:0005634",
  "gene_symbol": "STK11"
}